{
  "term_id": "GO:0098609",
  "gene_symbol": "SRPX2",
  "gene_name": "Sushi repeat-containing protein SRPX2",
  "term_label": "cell-cell adhesion",
  "gene": "UniProtKB:O60687"
}